{
  "term_label": "glucokinase activity",
  "gene_name": "Hexokinase-1",
  "term_id": "GO:0004340",
  "gene_symbol": "HK1",
  "gene": "UniProtKB:P19367"
}